{
  "gene": "UniProtKB:Q9NYW5",
  "term_label": "bitter taste receptor activity",
  "gene_name": "Taste receptor type 2 member 4",
  "term_id": "GO:0033038",
  "gene_symbol": "TAS2R4"
}